{
  "term_label": "Unknown molecular function",
  "gene_name": "Putative uncharacterized protein encoded by LINC00528",
  "gene": "UniProtKB:Q8N1L1",
  "gene_symbol": "LINC00528",
  "term_id": "UNKNOWN:0001"
}